{
  "gene": "UniProtKB:Q9NR46",
  "term_label": "membrane",
  "term_id": "GO:0016020",
  "gene_symbol": "SH3GLB2",
  "gene_name": "Endophilin-B2"
}